symbiont-mediated disruption of host anatomical structure [GO:0052111] (biological process) Relationships: is a type of GO:0141060 Subtypes: symbiont-mediated disruption of host cellular anatomical structure [GO:0052008], symbiont-mediated occlusion of host xylem [GO:0052112], symbiont-mediated disruption of host cuticle [GO:0085044], symbiont-mediated disruption of host tissue [GO:0141146] Definition: The process in which an organism effects a change that impairs the structure or function of an anatomical structure of the host organism. The host is defined as the larger of the organisms involved in a symbiotic interaction. Also known as: disruption by symbiont of host anatomical structure, modification by symbiont of host anatomical structure, cytopathogenic effect, modification by symbiont of host structure Sources: GOC:mtg_pamgo_17jul06